mammary placode formation [GO:0060596] (biological process) Regulation: positively regulated by positive regulation of mammary placode formation by mesenchymal-epithelial signaling [GO:0060617] Relationships: is a type of ectodermal placode formation [GO:0060788]; is part of mammary gland formation [GO:0060592] References: PMID:16168142 Sources: GOC:dph Definition: The developmental process in which the mammary placode forms. The mammary placode is a transient lens shaped structure that will give rise to the mammary bud proper.